{
  "term_id": "GO:0004594",
  "term_label": "pantothenate kinase activity",
  "gene_name": "Pantothenate kinase 3",
  "gene": "UniProtKB:Q9H999",
  "gene_symbol": "PANK3"
}